{
  "gene_symbol": "IGLC1",
  "gene_name": "Immunoglobulin lambda constant 1",
  "term_id": "GO:0071735",
  "term_label": "IgG immunoglobulin complex",
  "gene": "UniProtKB:P0CG04"
}